{
  "gene": "UniProtKB:Q9Y3R5",
  "gene_name": "Protein dopey-2",
  "gene_symbol": "DOP1B",
  "term_label": "endosome",
  "term_id": "GO:0005768"
}